{
  "term_label": "regulation of autophagy",
  "gene_name": "DNA damage-regulated autophagy modulator protein 2",
  "term_id": "GO:0010506",
  "gene_symbol": "DRAM2",
  "gene": "UniProtKB:Q6UX65"
}